{
  "gene_name": "1-phosphatidylinositol 4,5-bisphosphate phosphodiesterase zeta-1",
  "term_label": "phosphatidylinositol-4,5-bisphosphate phospholipase C activity",
  "term_id": "GO:0004435",
  "gene": "UniProtKB:Q86YW0",
  "gene_symbol": "PLCZ1"
}